{
  "term_label": "Unknown cellular component",
  "gene_symbol": "FOXD4",
  "gene_name": "Forkhead box protein D4",
  "gene": "UniProtKB:Q12950",
  "term_id": "UNKNOWN:0003"
}